{
  "term_id": "UNKNOWN:0001",
  "term_label": "Unknown molecular function",
  "gene_symbol": "KRTAP5-3",
  "gene_name": "Keratin-associated protein 5-3",
  "gene": "UniProtKB:Q6L8H2"
}